positive regulation of ATP-dependent activity [GO:0032781] (biological process) Definition: Any process that activates or increases the rate of an ATP-dependent activity. Relationships: is a type of regulation of ATP-dependent activity [GO:0043462]; is a type of positive regulation of molecular function [GO:0044093]; positively regulates GO:0140657 Also known as: positive regulation of ATPase activity, positive regulation of adenosinetriphosphatase activity, up regulation of ATPase activity, up-regulation of ATPase activity, upregulation of ATPase activity, activation of ATPase activity, stimulation of ATPase activity Sources: GOC:mah Subtypes: positive regulation of helicase activity [GO:0051096], positive regulation of ATPase-coupled calcium transmembrane transporter activity [GO:1901896], positive regulation of P-type sodium:potassium-exchanging transporter activity [GO:1903408], GO:1903612, positive regulation of DNA topoisomerase (ATP-hydrolyzing) activity [GO:2000373]